{
  "gene_symbol": "TMEM131",
  "term_label": "Unknown molecular function",
  "gene_name": "Transmembrane protein 131",
  "term_id": "UNKNOWN:0001",
  "gene": "UniProtKB:Q92545"
}